{
  "term_label": "postsynaptic density membrane",
  "gene_symbol": "DLG3",
  "gene": "UniProtKB:Q92796",
  "gene_name": "Disks large homolog 3",
  "term_id": "GO:0098839"
}